pyroptotic cell death [GO:0141201] (biological process) Relationships: is_a programmed cell death [GO:0012501]; is a type of pyroptotic inflammatory response [GO:0070269] Definition: A inflammatory cell death process associated with the generation of pyrogenic mediators that result from the activation of gasdermins. References: PMID:18846107, PMID:21760595, PMID:33883744 Subtypes: GO:1902483 Also known as: pyroptosis